{
  "gene_name": "Zinc finger protein 620",
  "gene_symbol": "ZNF620",
  "term_id": "GO:0000977",
  "term_label": "RNA polymerase II transcription regulatory region sequence-specific DNA binding",
  "gene": "UniProtKB:Q6ZNG0"
}